{
  "gene_symbol": "COX8C",
  "gene_name": "Cytochrome c oxidase subunit 8C, mitochondrial",
  "term_id": "UNKNOWN:0002",
  "gene": "UniProtKB:Q7Z4L0",
  "term_label": "Unknown biological process"
}